phosphate acetyltransferase activity [GO:0008959] (molecular function) Also known as: PTA, acetyl-CoA:phosphate acetyltransferase activity, phosphoacylase activity, phosphotransacetylase activity Relationships: is a type of acetyltransferase activity [GO:0016407] Definition: Catalysis of the reaction: acetyl-CoA + phosphate = CoA + acetyl phosphate. Sources: EC:2.3.1.8